{
  "gene_name": "Amyloid beta A4 precursor protein-binding family B member 1-interacting protein",
  "term_id": "GO:0030674",
  "term_label": "protein-macromolecule adaptor activity",
  "gene": "UniProtKB:Q7Z5R6",
  "gene_symbol": "APBB1IP"
}